{
  "term_label": "Unknown cellular component",
  "term_id": "UNKNOWN:0003",
  "gene_symbol": "CNMD",
  "gene": "UniProtKB:O75829",
  "gene_name": "Leukocyte cell-derived chemotaxin 1"
}